{
  "gene_name": "Zinc finger protein 446",
  "gene_symbol": "ZNF446",
  "term_label": "RNA polymerase II cis-regulatory region sequence-specific DNA binding",
  "term_id": "GO:0000978",
  "gene": "UniProtKB:Q9NWS9"
}